{
  "gene_symbol": "SYDE1",
  "gene": "UniProtKB:Q6ZW31",
  "term_id": "GO:0005096",
  "term_label": "GTPase activator activity",
  "gene_name": "Rho GTPase-activating protein SYDE1"
}